{
  "term_label": "heterochromatin formation",
  "gene_name": "Histone H2AX",
  "gene": "UniProtKB:P16104",
  "term_id": "GO:0031507",
  "gene_symbol": "H2AX"
}